{
  "gene": "UniProtKB:P40189",
  "term_id": "GO:0019221",
  "term_label": "cytokine-mediated signaling pathway",
  "gene_symbol": "IL6ST",
  "gene_name": "Interleukin-6 receptor subunit beta"
}